neuron projection membrane [GO:0032589] (CC) Sources: GOC:mah Definition: The portion of the plasma membrane surrounding a neuron projection. Subtypes: axolemma [GO:0030673], GO:0032590, GO:0032591, stereocilium membrane [GO:0060171] Relationships: is a type of cell projection membrane [GO:0031253]; is a type of leading edge membrane [GO:0031256]; is part of neuron projection [GO:0043005]